1,4-beta-D-xylan synthase activity [GO:0047517] (molecular function) Definition: Catalysis of the reaction: UDP-D-xylose + [(1->4)-beta-D-xylan](n) = UDP + [(1->4)-beta-D-xylan](n+1). Sources: EC:2.4.2.24 Also known as: 1,4-beta-xylan synthase activity, UDP-D-xylose:1,4-beta-D-xylan 4-beta-D-xylosyltransferase activity, uridine diphosphoxylose-1,4-beta-xylan xylosyltransferase activity, xylan synthase activity, xylan synthetase activity Relationships: is a type of UDP-glycosyltransferase activity [GO:0008194]; is a type of pentosyltransferase activity [GO:0016763]